{
  "term_id": "GO:0000981",
  "gene_symbol": "ZNF514",
  "gene_name": "Zinc finger protein 514",
  "term_label": "DNA-binding transcription factor activity, RNA polymerase II-specific",
  "gene": "UniProtKB:Q96K75"
}